methylglyoxal catabolic process to D-lactate via S-lactoyl-glutathione [GO:0019243] (biological process) References: PMID:2198020 Sources: GOC:ai, GOC:dph Relationships: is a type of methylglyoxal catabolic process to lactate [GO:0061727]; has part hydroxyacylglutathione hydrolase activity [GO:0004416]; has part lactoylglutathione lyase activity [GO:0004462] Definition: The chemical reactions and pathways resulting in the breakdown of methylglyoxal, CH3-CO-CHO, into D-lactate via the intermediate S-lactoyl-glutathione. Glutathione is used in the first step of the pathway and then regenerated in the second step. Also known as: D-lactate biosynthesis from methylglyoxal, D-lactate biosynthetic process from methylglyoxal, methylglyoxal breakdown to D-lactate, methylglyoxal degradation to D-lactate, methylglyoxal catabolism to D-lactate via S-lactoyl-glutathione, glyoxalase system, methylglyoxal detoxification